prolactin secretion [GO:0070459] (biological process) Sources: GOC:mah, ISBN:0198506732 Definition: The regulated release of prolactin, a peptide hormone that stimulates lactation, from secretory granules in the anterior pituitary. Regulation: negatively regulated by negative regulation of prolactin secretion [GO:1902721]; positively regulated by positive regulation of prolactin secretion [GO:1902722] Relationships: is a type of protein secretion [GO:0009306]; is a type of GO:0030072